{
  "gene": "UniProtKB:Q16563",
  "gene_symbol": "SYPL1",
  "term_label": "Unknown molecular function",
  "term_id": "UNKNOWN:0001",
  "gene_name": "Synaptophysin-like protein 1"
}